organophosphate:phosphate antiporter activity [GO:0015315] (molecular function) Subtypes: triose-phosphate:phosphate antiporter activity [GO:0009670], phosphoenolpyruvate:phosphate antiporter activity [GO:0015121], hexose-phosphate:phosphate antiporter activity [GO:0015526], glycerol-phosphate:phosphate antiporter activity [GO:0015527], glycerone phosphate:phosphate antiporter activity [GO:0051407], ATP:phosphate antiporter activity [GO:0140987], GO:0140988 Relationships: is a type of phosphate transmembrane transporter activity [GO:0005315]; is a type of solute:inorganic anion antiporter activity [GO:0005452] Also known as: organophosphate:inorganic phosphate antiporter activity Sources: TC:2.A.1.4.- Definition: Enables the transfer of a solute or solutes from one side of a membrane to the other according to the reaction: organophosphate(out) + phosphate(in) = organophosphate(in) +  phosphate(out).